{
  "term_id": "GO:0006357",
  "gene_symbol": "ATF5",
  "gene_name": "Cyclic AMP-dependent transcription factor ATF-5",
  "term_label": "regulation of transcription by RNA polymerase II",
  "gene": "UniProtKB:Q9Y2D1"
}